{
  "gene_symbol": "GTF2F1",
  "gene_name": "General transcription factor IIF subunit 1",
  "term_label": "transcription initiation at RNA polymerase II promoter",
  "gene": "UniProtKB:P35269",
  "term_id": "GO:0006367"
}